{
  "gene_symbol": "POT1",
  "gene_name": "Protection of telomeres protein 1",
  "gene": "UniProtKB:Q9NUX5",
  "term_id": "GO:0010521",
  "term_label": "telomerase inhibitor activity"
}